positive regulation of hexasaccharide transport [GO:1900299] (biological process) Also known as: up regulation of hexasaccharide transport, up-regulation of hexasaccharide transport, upregulation of hexasaccharide transport, activation of hexasaccharide transport Sources: GOC:TermGenie, GOC:mengo_curators Definition: Any process that activates or increases the frequency, rate or extent of hexasaccharide transport. Subtypes: positive regulation of maltohexaose transport [GO:1900314] Relationships: is a type of positive regulation of transport [GO:0051050]; is a type of GO:1900297; positively regulates hexasaccharide transport [GO:2001102]